{
  "term_label": "plasma membrane",
  "gene": "UniProtKB:Q6QNK2",
  "term_id": "GO:0005886",
  "gene_symbol": "ADGRD1",
  "gene_name": "Adhesion G-protein coupled receptor D1"
}